{
  "gene_symbol": "SSX8P",
  "term_id": "GO:0005634",
  "gene": "UniProtKB:Q7RTT4",
  "gene_name": "Putative protein SSX8",
  "term_label": "nucleus"
}